{
  "gene_name": "Serine_threonine-protein kinase Nek9",
  "gene": "UniProtKB:Q8TD19",
  "term_label": "mitotic cell cycle",
  "gene_symbol": "NEK9",
  "term_id": "GO:0000278"
}